negative regulation of maltoheptaose transport [GO:1900307] (biological process) Relationships: is a type of negative regulation of heptasaccharide transport [GO:1900295]; is a type of regulation of maltoheptaose transport [GO:1900306]; negatively regulates maltoheptaose transport [GO:2001105] Sources: GOC:TermGenie, GOC:mengo_curators Also known as: down regulation of maltoheptaose transport, down-regulation of maltoheptaose transport, downregulation of maltoheptaose transport, inhibition of maltoheptaose transport Definition: Any process that stops, prevents or reduces the frequency, rate or extent of maltoheptaose transport.